{
  "term_label": "RNA polymerase II, core complex",
  "gene_name": "DNA-directed RNA polymerase II subunit RPB1",
  "gene": "UniProtKB:P24928",
  "term_id": "GO:0005665",
  "gene_symbol": "POLR2A"
}